stress response to metal ion [GO:0097501] (biological process) Subtypes: stress response to copper ion [GO:1990169], stress response to cadmium ion [GO:1990170], stress response to zinc ion [GO:1990359], stress response to nickel ion [GO:1990532] Sources: GOC:kmv Relationships: is a type of GO:0006950; is_a response to metal ion [GO:0010038] Also known as: response to metal ion stress, response to excess metal ion, response to metal ion toxicity, response to metal toxicity Definition: Any process that results in a change in state or activity of a cell or an organism (in terms of movement, secretion, enzyme production, gene expression, etc.) as a result of a disturbance in organismal or cellular homeostasis caused by a metal ion stimulus.